{
  "gene_name": "Transcobalamin-2",
  "gene": "UniProtKB:P20062",
  "term_id": "GO:0015889",
  "gene_symbol": "TCN2",
  "term_label": "cobalamin transport"
}